APC-IQGAP complex [GO:0034743] (cellular component) Definition: A protein complex that contains the tumor suppressor protein adenomatous polyposis coli (APC) and the Rac1 and Cdc42 effector IQGAP1; may play a role in cytoskeleton organization and cell migration. References: PMID:15572129 Note: Note that the gene/protein name 'APC' should not be confused with the abbreviation for 'anaphase promoting complex'. Relationships: is a type of intracellular protein-containing complex [GO:0140535]; is a type of GTPase complex [GO:1905360]; BFO_0000050 cell leading edge [GO:0031252]